negative regulation of hepatic stellate cell activation [GO:2000490] (biological process) Relationships: is a type of negative regulation of cell activation [GO:0050866]; is a type of regulation of hepatic stellate cell activation [GO:2000489]; negatively regulates hepatic stellate cell activation [GO:0035733] Sources: GOC:obol Definition: Any process that stops, prevents or reduces the frequency, rate or extent of hepatic stellate cell activation.